{
  "gene_name": "Protein KHNYN",
  "term_label": "cytoplasmic ribonucleoprotein granule",
  "gene_symbol": "KHNYN",
  "term_id": "GO:0036464",
  "gene": "UniProtKB:O15037"
}